{
  "gene_symbol": "LCA5",
  "gene": "UniProtKB:Q86VQ0",
  "gene_name": "Lebercilin",
  "term_label": "Unknown molecular function",
  "term_id": "UNKNOWN:0001"
}